{
  "gene_name": "Cysteine and glycine-rich protein 2",
  "term_id": "GO:0030018",
  "gene": "UniProtKB:Q16527",
  "term_label": "Z disc",
  "gene_symbol": "CSRP2"
}